umami taste receptor activity [GO:0033042] (molecular function) Sources: GOC:mah Relationships: is_a GPCR taste receptor activity [GO:0090681]; is part of detection of chemical stimulus involved in sensory perception of umami taste [GO:0046535] Definition: Combining with soluble umami compounds to initiate a change in cell activity. These receptors are responsible for the sense of umami taste, the savory taste of meats and other foods that are rich in glutamates.